leptin-mediated signaling pathway [GO:0033210] (biological process) Subtypes: GO:0038108 Also known as: leptin-mediated signalling pathway, adipocytokine signaling pathway Sources: GOC:mah, GOC:signaling, GOC:yaf Definition: The series of molecular signals initiated by leptin binding to its receptor on the surface of a cell, and ending with the regulation of a downstream cellular process, e.g. transcription. Leptin is a hormone manufactured primarily in the adipocytes of white adipose tissue, and the level of circulating leptin is directly proportional to the total amount of fat in the body. Relationships: is a type of cytokine-mediated signaling pathway [GO:0019221]; is part of cellular response to leptin stimulus [GO:0044320]